{
  "gene_symbol": "ZNF91",
  "term_label": "nucleus",
  "gene": "UniProtKB:Q05481",
  "gene_name": "Zinc finger protein 91",
  "term_id": "GO:0005634"
}